{
  "gene": "UniProtKB:O75052",
  "gene_name": "Carboxyl-terminal PDZ ligand of neuronal nitric oxide synthase protein",
  "term_id": "GO:0050998",
  "gene_symbol": "NOS1AP",
  "term_label": "nitric-oxide synthase binding"
}